{
  "term_label": "IRE1-mediated unfolded protein response",
  "gene": "UniProtKB:O75460",
  "gene_name": "Serine_threonine-protein kinase_endoribonuclease IRE1",
  "term_id": "GO:0036498",
  "gene_symbol": "ERN1"
}